negative regulation of growth rate [GO:0045967] (biological process) Definition: Any process that reduces the rate of growth of all or part of an organism. Note: Note that this term and its definition depart from the usual conventions for GO 'regulation' process terms; regulation of rate is not usually distinguished from regulation of extent or frequency, but it makes sense to do so for growth regulation. Sources: GOC:mah Relationships: is a type of GO:0040009; is a type of negative regulation of growth [GO:0045926] Also known as: down regulation of growth rate, down-regulation of growth rate, downregulation of growth rate, inhibition of growth rate